{
  "term_id": "GO:0098632",
  "gene": "UniProtKB:Q8N6F1",
  "gene_name": "Claudin-19",
  "gene_symbol": "CLDN19",
  "term_label": "cell-cell adhesion mediator activity"
}